stigma development [GO:0048480] (biological process) Relationships: is a type of developmental process involved in reproduction [GO:0003006]; is a type of anatomical structure development [GO:0048856]; is part of GO:0048440 Sources: GOC:jid, PO:0009073 Definition: The process whose specific outcome is the progression of the stigma over time, from its formation to the mature structure. The stigma is the pollen-receptive surface of a carpel or group of fused carpels, usually sticky.